{
  "term_label": "immune response in nasopharyngeal-associated lymphoid tissue",
  "gene_name": "BPI fold-containing family A member 1",
  "term_id": "GO:0002395",
  "gene_symbol": "BPIFA1",
  "gene": "UniProtKB:Q9NP55"
}